{
  "term_id": "GO:0005158",
  "gene": "UniProtKB:F8WCM5",
  "gene_name": "Insulin, isoform 2",
  "gene_symbol": "INS-IGF2",
  "term_label": "insulin receptor binding"
}